{
  "term_id": "GO:0048468",
  "gene_name": "Iroquois-class homeodomain protein IRX-4",
  "term_label": "cell development",
  "gene_symbol": "IRX4",
  "gene": "UniProtKB:P78413"
}